{
  "term_label": "DNA-binding transcription activator activity, RNA polymerase II-specific",
  "gene_name": "PR domain zinc finger protein 15",
  "gene": "UniProtKB:P57071",
  "gene_symbol": "PRDM15",
  "term_id": "GO:0001228"
}